{
  "gene_name": "Cyclin-dependent kinase 4 inhibitor B",
  "term_id": "GO:0004861",
  "gene": "UniProtKB:P42772",
  "term_label": "cyclin-dependent protein serine/threonine kinase inhibitor activity",
  "gene_symbol": "CDKN2B"
}